Ssh1 translocon complex [GO:0071261] (cellular component) References: PMID:12134063, PMID:8612571 Sources: GOC:mah Relationships: is a type of translocon complex [GO:0071256] Definition: A translocon complex that contains a core heterotrimer of alpha, beta and gamma subunits, and may contain additional proteins (translocon-associated proteins or TRAPs); in budding yeast the core proteins are Ssh1p, Sbh2p, and Sss1p. The Ssh1 translocon complex is involved in the cotranslational pathway of protein transport across the ER membrane, and recognizes proteins bearing strongly hydrophobic signal sequences. Also known as: Ssh1p-Sss1p-Sbh2p complex